{
  "gene": "UniProtKB:Q6V1P9",
  "gene_symbol": "DCHS2",
  "term_id": "GO:0007409",
  "gene_name": "Protocadherin-23",
  "term_label": "axonogenesis"
}